oligodendrocyte cell fate commitment [GO:0021779] (biological process) Sources: GOC:cls, GOC:dgh, GOC:dph, GOC:jid, GO_REF:0000021 Relationships: is a type of glial cell fate commitment [GO:0021781]; is a type of GO:0048709 Definition: The process in which the developmental fate of a cell becomes restricted such that it will develop into an oligodendrocyte.